{
  "gene": "UniProtKB:Q13323",
  "term_label": "Unknown cellular component",
  "term_id": "UNKNOWN:0003",
  "gene_name": "Bcl-2-interacting killer",
  "gene_symbol": "BIK"
}